{
  "gene_name": "CBP80_20-dependent translation initiation factor",
  "gene_symbol": "CTIF",
  "gene": "UniProtKB:O43310",
  "term_id": "GO:0006446",
  "term_label": "regulation of translational initiation"
}